{
  "gene_symbol": "CYP4F22",
  "term_label": "ceramide biosynthetic process",
  "term_id": "GO:0046513",
  "gene_name": "Ultra-long-chain fatty acid omega-hydroxylase",
  "gene": "UniProtKB:Q6NT55"
}